{
  "term_label": "RNA polymerase II cis-regulatory region sequence-specific DNA binding",
  "gene": "UniProtKB:Q9UL49",
  "gene_name": "Transcription factor-like 5 protein",
  "term_id": "GO:0000978",
  "gene_symbol": "TCFL5"
}